positive chemotaxis [GO:0050918] (biological process) Relationships: is a type of chemotaxis [GO:0006935] Sources: GOC:ai, GOC:bf, GOC:isa_complete Also known as: chemoattraction Subtypes: pollen tube guidance [GO:0010183], synaptic target attraction [GO:0016200], chemoattraction involved in embryonic olfactory bulb interneuron precursor migration [GO:0021835], chemoattraction involved in interneuron migration from the subpallium to the cortex [GO:0021841], GO:0021951, germ cell attraction [GO:0035232], positive aerotaxis [GO:0052131], chemoattraction of axon [GO:0061642] Regulation: regulated by GO:0050926; positively regulated by positive regulation of positive chemotaxis [GO:0050927]; negatively regulated by negative regulation of positive chemotaxis [GO:0050928] Definition: The directed movement of a motile cell or organism towards a higher concentration of a chemical.